{
  "term_label": "cell surface receptor protein serine/threonine kinase signaling pathway",
  "gene": "UniProtKB:P55107",
  "term_id": "GO:0007178",
  "gene_name": "Growth_differentiation factor 10",
  "gene_symbol": "GDF10"
}